{
  "gene": "UniProtKB:P60507",
  "gene_name": "Endogenous retrovirus group FC1 Env polyprotein",
  "term_label": "Unknown cellular component",
  "term_id": "UNKNOWN:0003",
  "gene_symbol": "ERVFC1"
}